meiotic sister chromatid separation [GO:0051757] (BP) Also known as: meiotic sister chromatid resolution Definition: The process in which sister chromatids are physically detached from each other during meiosis. Relationships: is a type of meiotic chromosome separation [GO:0051307] References: PMID:14730319, PMID:16325576 Sources: GOC:ai